propionate transmembrane transporter activity [GO:0015552] (molecular function) Relationships: is a type of short-chain fatty acid transmembrane transporter activity [GO:0015636]; is part of propanoate transmembrane transport [GO:0015730] Subtypes: GO:0015544 Sources: GOC:ai Definition: Enables the transfer of propionate from one side of a membrane to the other. Propionate (or propanoate) is the organic acid CH3-CH2-COOH.